{
  "gene_symbol": "AP2S1",
  "term_id": "UNKNOWN:0003",
  "gene_name": "AP-2 complex subunit sigma",
  "term_label": "Unknown cellular component",
  "gene": "UniProtKB:P53680"
}